{
  "gene_name": "NUT family member 2B",
  "term_id": "UNKNOWN:0001",
  "gene": "UniProtKB:A6NNL0",
  "gene_symbol": "NUTM2B",
  "term_label": "Unknown molecular function"
}